{
  "term_label": "estrogen metabolic process",
  "gene": "UniProtKB:O75310",
  "gene_symbol": "UGT2B11",
  "term_id": "GO:0008210",
  "gene_name": "UDP-glucuronosyltransferase 2B11"
}